{
  "gene_symbol": "STX10",
  "term_id": "GO:0006906",
  "term_label": "vesicle fusion",
  "gene": "UniProtKB:O60499",
  "gene_name": "Syntaxin-10"
}